{
  "term_id": "GO:0009395",
  "gene_symbol": "PLD1",
  "gene": "UniProtKB:Q13393",
  "gene_name": "Phospholipase D1",
  "term_label": "phospholipid catabolic process"
}